{
  "term_id": "GO:0000987",
  "term_label": "cis-regulatory region sequence-specific DNA binding",
  "gene_symbol": "JMJD8",
  "gene_name": "JmjC domain-containing protein 8",
  "gene": "UniProtKB:Q96S16"
}